microtubule plus end polymerase [GO:0061863] (molecular function) Definition: Catalysis of the transfer of tubulin dimers to the plus end of a microtubule. The reaction is reversible depending on the availability of dimers. References: PMID:27872152 Relationships: is a type of transferase activity [GO:0016740]; is_a catalytic activity, acting on a protein [GO:0140096]; is part of microtubule cytoskeleton organization [GO:0000226]